{
  "gene_symbol": "TRAJ20",
  "gene_name": "T cell receptor alpha joining 20 (Fragment)",
  "term_id": "UNKNOWN:0001",
  "term_label": "Unknown molecular function",
  "gene": "UniProtKB:A0A075B6Z1"
}